{
  "gene_name": "Protein SPATA31F3",
  "term_label": "Unknown biological process",
  "gene": "UniProtKB:A6NFA0",
  "term_id": "UNKNOWN:0002",
  "gene_symbol": "SPATA31F3"
}